{
  "gene": "UniProtKB:Q86WS3",
  "gene_name": "Oocyte-secreted protein 2",
  "gene_symbol": "OOSP2",
  "term_label": "Unknown cellular component",
  "term_id": "UNKNOWN:0003"
}